{
  "gene": "UniProtKB:Q6UXS9",
  "gene_name": "Inactive caspase-12",
  "term_label": "positive regulation of inflammatory response",
  "gene_symbol": "CASP12",
  "term_id": "GO:0050729"
}